{
  "term_id": "GO:0006883",
  "gene_name": "Potassium-transporting ATPase alpha chain 2",
  "term_label": "intracellular sodium ion homeostasis",
  "gene_symbol": "ATP12A",
  "gene": "UniProtKB:P54707"
}